response to platelet aggregation inhibitor [GO:0061478] (BP) Definition: Any process that results in a change in state or activity of a cell or an organism (in terms of movement, secretion, enzyme production, gene expression, etc.) as a result of a platelet aggregation inhibitor stimulus. Relationships: is a type of GO:0042221 Sources: GOC:dph